{
  "gene_name": "Opioid growth factor receptor-like protein 1",
  "term_id": "UNKNOWN:0002",
  "gene": "UniProtKB:Q5TC84",
  "gene_symbol": "OGFRL1",
  "term_label": "Unknown biological process"
}